{
  "gene_symbol": "CXCR1",
  "gene": "UniProtKB:P25024",
  "term_label": "positive regulation of cytosolic calcium ion concentration",
  "term_id": "GO:0007204",
  "gene_name": "C-X-C chemokine receptor type 1"
}